{
  "gene_name": "Nuclear receptor subfamily 4 group A member 1",
  "term_id": "GO:0000978",
  "gene": "UniProtKB:P22736",
  "gene_symbol": "NR4A1",
  "term_label": "RNA polymerase II cis-regulatory region sequence-specific DNA binding"
}